{
  "term_id": "GO:0050501",
  "gene_name": "Hyaluronan synthase 2",
  "gene": "UniProtKB:Q92819",
  "term_label": "hyaluronan synthase activity",
  "gene_symbol": "HAS2"
}